negative regulation of endoplasmic reticulum unfolded protein response [GO:1900102] (biological process) Sources: GOC:TermGenie Subtypes: GO:1903892, negative regulation of IRE1-mediated unfolded protein response [GO:1903895], negative regulation of PERK-mediated unfolded protein response [GO:1903898] Relationships: is_a regulation of endoplasmic reticulum unfolded protein response [GO:1900101]; is a type of negative regulation of intracellular signal transduction [GO:1902532]; is a type of negative regulation of response to endoplasmic reticulum stress [GO:1903573]; negatively regulates GO:0030968 Definition: Any process that stops, prevents or reduces the frequency, rate or extent of endoplasmic reticulum unfolded protein response. Also known as: down regulation of ER unfolded protein response, down regulation of endoplasmic reticulum unfolded protein response, down regulation of erUPR, down-regulation of ER unfolded protein response, down-regulation of endoplasmic reticulum unfolded protein response, down-regulation of erUPR, downregulation of ER unfolded protein response, downregulation of endoplasmic reticulum unfolded protein response, downregulation of erUPR, inhibition of ER unfolded protein response, inhibition of erUPR, negative regulation of ER unfolded protein response, negative regulation of erUPR, inhibition of endoplasmic reticulum unfolded protein response, down regulation of SREBP-mediated signalling pathway, down-regulation of SREBP-mediated signalling pathway, downregulation of SREBP-mediated signalling pathway, inhibition of SREBP-mediated signalling pathway, negative regulation of SREBP-mediated signalling pathway